{
  "term_label": "extracellular space",
  "gene": "UniProtKB:Q14767",
  "term_id": "GO:0005615",
  "gene_symbol": "LTBP2",
  "gene_name": "Latent-transforming growth factor beta-binding protein 2"
}